{
  "term_label": "Unknown cellular component",
  "gene": "UniProtKB:A6NIN4",
  "gene_name": "RING finger protein 227",
  "gene_symbol": "RNF227",
  "term_id": "UNKNOWN:0003"
}